linear vestibuloocular reflex [GO:0060007] (biological process) References: PMID:11784757 Sources: GOC:dph Definition: A vestibular reflex by which a response to a linear acceleration stimulus begins with an afferent nerve impulse from a receptor in the otolith and ends with the compensatory action of eye muscles. Signaling never reaches a level of consciousness. Relationships: is a type of vestibular reflex [GO:0060005]